{
  "term_label": "adenylate cyclase-activating G protein-coupled receptor signaling pathway",
  "gene_symbol": "ADGRF1",
  "term_id": "GO:0007189",
  "gene_name": "Adhesion G-protein coupled receptor F1",
  "gene": "UniProtKB:Q5T601"
}